regulation of amyloid precursor protein biosynthetic process [GO:0042984] (biological process) Definition: Any process that modulates the frequency, rate or extent of the chemical reactions and pathways resulting in the formation of amyloid precursor protein (APP), the precursor of amyloid-beta. Sources: GOC:go_curators Also known as: regulation of APP biosynthesis, regulation of APP biosynthetic process, regulation of amyloid precursor protein anabolism, regulation of amyloid precursor protein biosynthesis, regulation of amyloid precursor protein formation, regulation of amyloid precursor protein synthesis Relationships: is a type of GO:0010559; regulates amyloid precursor protein biosynthetic process [GO:0042983] Subtypes: negative regulation of amyloid precursor protein biosynthetic process [GO:0042985], GO:0042986